dendrite self-avoidance [GO:0070593] (biological process) Definition: The process in which dendrites recognize and avoid contact with sister dendrites from the same cell. Also known as: dendrite repulsion References: PMID:17482551 Sources: GOC:sart Relationships: is_a neuron recognition [GO:0008038]